{
  "term_label": "glycerophospholipid catabolic process",
  "gene": "UniProtKB:Q86XP0",
  "term_id": "GO:0046475",
  "gene_name": "Cytosolic phospholipase A2 delta",
  "gene_symbol": "PLA2G4D"
}